{
  "gene_name": "Gamma-tubulin complex component 3",
  "term_id": "GO:0000278",
  "gene": "UniProtKB:Q96CW5",
  "gene_symbol": "TUBGCP3",
  "term_label": "mitotic cell cycle"
}